positive regulation of tonic skeletal muscle contraction [GO:0014747] (BP) Sources: GOC:ef, GOC:mtg_muscle Definition: Any process that activates or increases the frequency, rate or extent of tonic skeletal muscle contraction. Relationships: is a type of regulation of tonic skeletal muscle contraction [GO:0014746]; is a type of positive regulation of striated muscle contraction [GO:0045989]; positively regulates tonic skeletal muscle contraction [GO:0014720]